{
  "term_label": "cytoplasm",
  "gene_name": "KN motif and ankyrin repeat domain-containing protein 4",
  "term_id": "GO:0005737",
  "gene": "UniProtKB:Q5T7N3",
  "gene_symbol": "KANK4"
}